{
  "term_id": "GO:0019901",
  "gene_name": "POTE ankyrin domain family member F",
  "gene_symbol": "POTEF",
  "gene": "UniProtKB:A5A3E0",
  "term_label": "protein kinase binding"
}